terpenoid indole alkaloid biosynthetic process [GO:0009709] (biological process) Subtypes: ergot alkaloid biosynthetic process [GO:0035837], paxilline biosynthetic process [GO:0140873], vindoline biosynthetic process [GO:1900985], GO:1900988 Sources: GOC:ai, http://rycomusa.com/aspp2000/public/P29/0525.html Also known as: terpenoid indole alkaloid anabolism, terpenoid indole alkaloid biosynthesis, terpenoid indole alkaloid formation, terpenoid indole alkaloid synthesis Relationships: is a type of indole alkaloid biosynthetic process [GO:0035835]; is a type of terpenoid indole alkaloid metabolic process [GO:0046447] Definition: The chemical reactions and pathways resulting in the formation of terpenoid indole alkaloids, compounds formed from the condensation of tryptamine (derived from tryptophan) and secologanin (derived from geranyl pyrophosphate).